{
  "gene_name": "Disintegrin and metalloproteinase domain-containing protein 8",
  "term_id": "GO:0002693",
  "term_label": "positive regulation of cellular extravasation",
  "gene_symbol": "ADAM8",
  "gene": "UniProtKB:P78325"
}